{
  "term_label": "Unknown biological process",
  "gene_symbol": "SPATA20",
  "gene_name": "Spermatogenesis-associated protein 20",
  "term_id": "UNKNOWN:0002",
  "gene": "UniProtKB:Q8TB22"
}